{
  "term_label": "gap junction channel activity",
  "gene_symbol": "GJA1",
  "gene_name": "Gap junction alpha-1 protein",
  "term_id": "GO:0005243",
  "gene": "UniProtKB:P17302"
}